{
  "gene": "UniProtKB:Q13492",
  "gene_name": "Phosphatidylinositol-binding clathrin assembly protein",
  "term_label": "clathrin-dependent endocytosis",
  "gene_symbol": "PICALM",
  "term_id": "GO:0072583"
}